regulation of locomotion involved in locomotory behavior [GO:0090325] (biological process) Definition: Any process that modulates the frequency, rate, or extent of the self-propelled movement of a cell or organism from one location to another in a behavioral context; the aspect of locomotory behavior having to do with movement. Subtypes: GO:0090326, negative regulation of locomotion involved in locomotory behavior [GO:0090327] Sources: GOC:dph, GOC:kmv, GOC:tb Relationships: is a type of regulation of locomotion [GO:0040012]; is a type of regulation of behavior [GO:0050795]; regulates locomotion involved in locomotory behavior [GO:0031987]